oral apparatus [GO:0031912] (cellular component) Definition: Complex basket- or funnel-like structure used by the cell to collect food and channel it to the cytostome; includes specialized sub-structures made up of closely-spaced cilia and underlying basal bodies and fibrillar systems. Note: Note that this term refers to a subcellular structure characteristic of ciliate protozoans, and should not be confused with oral anatomical structures of multicellular animals. Relationships: is a type of GO:0110165 References: PMID:10503189